cardiolipin binding [GO:1901612] (molecular function) Sources: GOC:TermGenie, GOC:kmv Definition: Binding to cardiolipin. Relationships: is a type of phosphatidylglycerol binding [GO:1901611]